thymine binding [GO:0002059] (MF) Relationships: is a type of pyrimidine nucleobase binding [GO:0002061] Definition: Binding to thymine. Sources: GOC:hjd